RNA polymerase V transcription regulator complex [GO:0090578] (cellular component) Definition: A transcription factor complex that acts at a regulatory region of a gene transcribed by RNA polymerase V. Also known as: RNA polymerase V transcription factor complex Sources: GOC:tb Relationships: is a type of transcription regulator complex [GO:0005667]